{
  "gene": "UniProtKB:P08476",
  "term_label": "cell surface receptor protein serine/threonine kinase signaling pathway",
  "term_id": "GO:0007178",
  "gene_symbol": "INHBA",
  "gene_name": "Inhibin beta A chain"
}